{
  "gene": "UniProtKB:A6NMS3",
  "gene_symbol": "OR5K4",
  "gene_name": "Olfactory receptor 5K4",
  "term_id": "GO:0004984",
  "term_label": "olfactory receptor activity"
}